{
  "gene": "UniProtKB:Q6PEX3",
  "term_id": "UNKNOWN:0003",
  "gene_name": "Keratin-associated protein 26-1",
  "gene_symbol": "KRTAP26-1",
  "term_label": "Unknown cellular component"
}